{
  "term_label": "apoptotic process",
  "term_id": "GO:0006915",
  "gene_name": "Caspase-7",
  "gene": "UniProtKB:P55210",
  "gene_symbol": "CASP7"
}